T=219 icosahedral capsid [GO:0039629] (CC) Sources: GOC:plm, UniProtKB-KW:KW-1151 Relationships: is a type of icosahedral viral capsid [GO:0019030] Definition: The protein coat that surrounds the infective nucleic acid in some virus particles where the subunits (capsomeres) are arranged to form an icosahedron with T=219 symmetry. T=219 icosahedral capsid is composed of 12 pentameric and 2180 hexameric capsomeres for a total of 13140 capsid proteins.